{
  "gene_symbol": "FGF21",
  "term_id": "GO:0022008",
  "term_label": "neurogenesis",
  "gene": "UniProtKB:Q9NSA1",
  "gene_name": "Fibroblast growth factor 21"
}